{
  "term_label": "intracellular signal transduction",
  "term_id": "GO:0035556",
  "gene_name": "Leucine-rich repeat-containing protein 59",
  "gene_symbol": "LRRC59",
  "gene": "UniProtKB:Q96AG4"
}